{
  "gene_name": "Acid-sensing ion channel 3",
  "gene_symbol": "ASIC3",
  "term_id": "GO:0035725",
  "gene": "UniProtKB:Q9UHC3",
  "term_label": "sodium ion transmembrane transport"
}